{
  "term_id": "UNKNOWN:0001",
  "gene_name": "RNA-binding protein with serine-rich domain 1",
  "term_label": "Unknown molecular function",
  "gene": "UniProtKB:Q15287",
  "gene_symbol": "RNPS1"
}